{
  "gene": "UniProtKB:Q8NCG7",
  "term_label": "plasma membrane",
  "gene_symbol": "DAGLB",
  "term_id": "GO:0005886",
  "gene_name": "Diacylglycerol lipase-beta"
}